corticospinal neuron axon guidance through the medullary pyramid [GO:0021971] (biological process) Definition: The process in which the migration of an axon growth cone of a pyramidal cell that is part of the corticospinal tract is directed after exiting the basilar pons through the medullary pyramid in response to a combination of attractive and repulsive cues. Also known as: corticospinal neuron axon pathfinding through the medullary pyramid References: PMID:9878731 Sources: GOC:cls, GOC:dgh, GOC:dph, GOC:jid, GO_REF:0000021 Relationships: is a type of GO:0007411; is part of corticospinal neuron axon guidance [GO:0021966]